acute inflammatory response to non-antigenic stimulus [GO:0002525] (biological process) Regulation: regulated by regulation of acute inflammatory response to non-antigenic stimulus [GO:0002877]; negatively regulated by negative regulation of acute inflammatory response to non-antigenic stimulus [GO:0002878]; positively regulated by positive regulation of acute inflammatory response to non-antigenic stimulus [GO:0002879] Relationships: is a type of acute inflammatory response [GO:0002526] Definition: An acute inflammatory response to non-antigenic stimuli such as heat or physical trauma. References: PMID:16459497, PMID:9073326 Sources: GOC:jal